{
  "gene": "UniProtKB:P0CJ90",
  "term_label": "DNA-binding transcription factor activity, RNA polymerase II-specific",
  "term_id": "GO:0000981",
  "gene_name": "Double homeobox protein 4-like protein 7",
  "gene_symbol": "DUX4L7"
}